extracellular matrix structural constituent [GO:0005201] (molecular function) Also known as: core extracellular matrix, core matrisome, extracellular matrix glycoprotein Relationships: is a type of GO:0005198; occurs in extracellular matrix [GO:0031012] Subtypes: extracellular matrix structural constituent conferring tensile strength [GO:0030020], extracellular matrix structural constituent conferring compression resistance [GO:0030021], extracellular matrix constituent conferring elasticity [GO:0030023], extracellular matrix constituent, lubricant activity [GO:0030197], structural constituent of egg coat [GO:0035804], structural constituent of synapse-associated extracellular matrix [GO:0150043] Definition: The action of a molecule that contributes to the structural integrity of the extracellular matrix. Note: Extracellular matrix glycoproteins may be annotated to this term. PMID:24443019 Sources: GOC:mah